{
  "gene_symbol": "TRBJ1-3",
  "gene_name": "T cell receptor beta joining 1-3",
  "gene": "UniProtKB:A0A0J9YWP8",
  "term_label": "Unknown molecular function",
  "term_id": "UNKNOWN:0001"
}